{
  "term_id": "GO:0005886",
  "gene": "UniProtKB:O43921",
  "gene_symbol": "EFNA2",
  "gene_name": "Ephrin-A2",
  "term_label": "plasma membrane"
}